negative regulation of homophilic cell adhesion [GO:1903386] (biological process) Also known as: down regulation of homophilic cell adhesion, down-regulation of homophilic cell adhesion, downregulation of homophilic cell adhesion, inhibition of homophilic cell adhesion Relationships: is a type of GO:0022408; is a type of GO:1903385; negatively regulates homophilic cell-cell adhesion [GO:0007156] Definition: Any process that stops, prevents or reduces the frequency, rate or extent of homophilic cell adhesion. References: PMID:21724833 Sources: GOC:TermGenie, GOC:als, GO_REF:0000058